{
  "gene_name": "Alcohol dehydrogenase class-3",
  "term_label": "S-(hydroxymethyl)glutathione dehydrogenase [NAD(P)+] activity",
  "gene_symbol": "ADH5",
  "term_id": "GO:0051903",
  "gene": "UniProtKB:P11766"
}